{
  "term_id": "UNKNOWN:0001",
  "term_label": "Unknown molecular function",
  "gene_name": "Coagulation factor VII",
  "gene_symbol": "F7",
  "gene": "UniProtKB:P08709"
}